negative regulation of mismatch repair [GO:0032424] (biological process) Sources: GOC:vk Definition: Any process that stops, prevents, or reduces the frequency, rate or extent of mismatch repair. Also known as: down regulation of mismatch repair, down-regulation of mismatch repair, downregulation of mismatch repair, inhibition of mismatch repair Relationships: is_a GO:0032423; is a type of negative regulation of DNA repair [GO:0045738]; negatively regulates mismatch repair [GO:0006298]